{
  "term_id": "GO:0016323",
  "gene_name": "Solute carrier organic anion transporter family member 3A1",
  "gene_symbol": "SLCO3A1",
  "term_label": "basolateral plasma membrane",
  "gene": "UniProtKB:Q9UIG8"
}